{
  "gene": "UniProtKB:A0A075B6Y8",
  "term_label": "Unknown molecular function",
  "gene_symbol": "TRAJ11",
  "term_id": "UNKNOWN:0001",
  "gene_name": "T cell receptor alpha joining 11 (Fragment)"
}